{
  "term_id": "UNKNOWN:0001",
  "gene_name": "Proline-rich transmembrane protein 2",
  "gene": "UniProtKB:Q7Z6L0",
  "gene_symbol": "PRRT2",
  "term_label": "Unknown molecular function"
}